{
  "term_id": "UNKNOWN:0002",
  "term_label": "Unknown biological process",
  "gene": "UniProtKB:Q9NW82",
  "gene_symbol": "WDR70",
  "gene_name": "WD repeat-containing protein 70"
}